{
  "gene": "UniProtKB:Q5D0E6",
  "term_label": "tRNA C3-cytosine methylation",
  "gene_symbol": "DALRD3",
  "term_id": "GO:0106217",
  "gene_name": "DALR anticodon-binding domain-containing protein 3"
}